regulation of ketone catabolic process [GO:0010567] (biological process) Relationships: is a type of regulation of catabolic process [GO:0009894]; is a type of GO:0010565; is a type of regulation of small molecule metabolic process [GO:0062012]; regulates ketone catabolic process [GO:0042182] Definition: Any process that modulates the frequency, rate or extent of the chemical reactions and pathways resulting in the breakdown of a ketone, carried out by individual cells. Sources: GOC:dph, GOC:tb